{
  "term_id": "GO:0071735",
  "term_label": "IgG immunoglobulin complex",
  "gene_symbol": "IGLL1",
  "gene_name": "Immunoglobulin lambda-like polypeptide 1",
  "gene": "UniProtKB:P15814"
}